{
  "term_id": "GO:0042162",
  "term_label": "telomeric DNA binding",
  "gene": "UniProtKB:P13010",
  "gene_symbol": "XRCC5",
  "gene_name": "X-ray repair cross-complementing protein 5"
}